{
  "gene_name": "Adhesion G protein-coupled receptor E5",
  "term_label": "plasma membrane",
  "term_id": "GO:0005886",
  "gene": "UniProtKB:P48960",
  "gene_symbol": "ADGRE5"
}